{
  "gene": "UniProtKB:Q06945",
  "gene_symbol": "SOX4",
  "term_label": "brain development",
  "term_id": "GO:0007420",
  "gene_name": "Transcription factor SOX-4"
}